{
  "gene": "UniProtKB:Q8TAQ2",
  "gene_symbol": "SMARCC2",
  "gene_name": "SWI_SNF complex subunit SMARCC2",
  "term_id": "GO:0016514",
  "term_label": "SWI/SNF complex"
}